{
  "term_label": "COPI vesicle coat",
  "term_id": "GO:0030126",
  "gene_symbol": "COPE",
  "gene_name": "Coatomer subunit epsilon",
  "gene": "UniProtKB:O14579"
}